{
  "gene_symbol": "SLC4A11",
  "term_label": "transmembrane transporter activity",
  "gene": "UniProtKB:Q8NBS3",
  "gene_name": "Solute carrier family 4 member 11",
  "term_id": "GO:0022857"
}